{
  "gene_name": "Tyrosine-protein kinase CSK",
  "term_label": "adherens junction organization",
  "term_id": "GO:0034332",
  "gene": "UniProtKB:P41240",
  "gene_symbol": "CSK"
}